{
  "term_id": "GO:0005882",
  "gene": "UniProtKB:P07197",
  "gene_name": "Neurofilament medium polypeptide",
  "term_label": "intermediate filament",
  "gene_symbol": "NEFM"
}